{
  "term_id": "GO:0004386",
  "gene_symbol": "DHX34",
  "gene_name": "Probable ATP-dependent RNA helicase DHX34",
  "term_label": "helicase activity",
  "gene": "UniProtKB:Q14147"
}